{
  "term_id": "GO:0008378",
  "gene_name": "Beta-1,4-galactosyltransferase 2",
  "gene_symbol": "B4GALT2",
  "gene": "UniProtKB:O60909",
  "term_label": "galactosyltransferase activity"
}